{
  "gene_name": "T-box transcription factor TBX22",
  "gene": "UniProtKB:Q9Y458",
  "gene_symbol": "TBX22",
  "term_id": "GO:0000981",
  "term_label": "DNA-binding transcription factor activity, RNA polymerase II-specific"
}